{
  "gene_name": "Myosin regulatory light chain 11",
  "gene": "UniProtKB:Q96A32",
  "term_id": "GO:0005737",
  "term_label": "cytoplasm",
  "gene_symbol": "MYL11"
}